{
  "term_id": "GO:0045766",
  "gene_name": "Vascular endothelial growth factor receptor 2",
  "gene": "UniProtKB:P35968",
  "gene_symbol": "KDR",
  "term_label": "positive regulation of angiogenesis"
}